{
  "term_label": "positive regulation of protein targeting to membrane",
  "gene_symbol": "TCAF2C",
  "term_id": "GO:0090314",
  "gene": "UniProtKB:A0A1B0GVM2",
  "gene_name": "TRPM8 channel associated factor 2C (Fragment)"
}